{
  "gene_name": "5-hydroxytryptamine receptor 3D",
  "gene": "UniProtKB:Q70Z44",
  "term_id": "GO:0034220",
  "term_label": "monoatomic ion transmembrane transport",
  "gene_symbol": "HTR3D"
}